{
  "gene_symbol": "IL2RA",
  "term_id": "GO:0006954",
  "term_label": "inflammatory response",
  "gene": "UniProtKB:P01589",
  "gene_name": "Interleukin-2 receptor subunit alpha"
}